{
  "term_label": "galactose catabolic process via UDP-galactose, Leloir pathway",
  "gene_symbol": "GALT",
  "gene": "UniProtKB:P07902",
  "gene_name": "Galactose-1-phosphate uridylyltransferase",
  "term_id": "GO:0033499"
}